{
  "gene_name": "5-hydroxytryptamine receptor 4",
  "term_label": "plasma membrane",
  "term_id": "GO:0005886",
  "gene": "UniProtKB:Q13639",
  "gene_symbol": "HTR4"
}